{
  "gene_symbol": "VN1R3",
  "term_label": "pheromone binding",
  "gene": "UniProtKB:Q9BXE9",
  "gene_name": "Vomeronasal type-1 receptor 3",
  "term_id": "GO:0005550"
}